{
  "gene_name": "Centromere protein Q",
  "gene_symbol": "CENPQ",
  "term_label": "nucleus",
  "gene": "UniProtKB:Q7L2Z9",
  "term_id": "GO:0005634"
}